{
  "gene_symbol": "HNRNPA1",
  "gene": "UniProtKB:P09651",
  "term_id": "GO:0003730",
  "term_label": "mRNA 3'-UTR binding",
  "gene_name": "Heterogeneous nuclear ribonucleoprotein A1"
}